{
  "term_label": "Unknown biological process",
  "gene_name": "BPI fold-containing family A member 3",
  "gene": "UniProtKB:Q9BQP9",
  "gene_symbol": "BPIFA3",
  "term_id": "UNKNOWN:0002"
}